{
  "gene_symbol": "TNC",
  "gene": "UniProtKB:P24821",
  "term_label": "extracellular space",
  "term_id": "GO:0005615",
  "gene_name": "Tenascin"
}